{
  "gene_name": "Voltage-dependent L-type calcium channel subunit beta-1",
  "term_id": "GO:0006816",
  "term_label": "calcium ion transport",
  "gene": "UniProtKB:Q02641",
  "gene_symbol": "CACNB1"
}